{
  "term_label": "protein folding",
  "gene_symbol": "DNAJB12",
  "gene": "UniProtKB:Q9NXW2",
  "gene_name": "DnaJ homolog subfamily B member 12",
  "term_id": "GO:0006457"
}